{
  "gene_symbol": "TSSC4",
  "gene_name": "U5 small nuclear ribonucleoprotein TSSC4",
  "term_label": "spliceosomal tri-snRNP complex assembly",
  "gene": "UniProtKB:Q9Y5U2",
  "term_id": "GO:0000244"
}